{
  "gene_name": "Tetratricopeptide repeat protein 12",
  "gene": "UniProtKB:Q9H892",
  "gene_symbol": "TTC12",
  "term_id": "GO:0005813",
  "term_label": "centrosome"
}